{
  "gene": "UniProtKB:Q96S44",
  "gene_name": "EKC_KEOPS complex subunit TP53RK",
  "gene_symbol": "TP53RK",
  "term_id": "GO:0070525",
  "term_label": "tRNA threonylcarbamoyladenosine metabolic process"
}